{
  "gene": "UniProtKB:Q8N135",
  "gene_symbol": "LGI4",
  "gene_name": "Leucine-rich repeat LGI family member 4",
  "term_id": "UNKNOWN:0001",
  "term_label": "Unknown molecular function"
}